T cell differentiation [GO:0030217] (biological process) Subtypes: T cell differentiation involved in immune response [GO:0002292], T cell differentiation in thymus [GO:0033077], extrathymic T cell differentiation [GO:0033078], gamma-delta T cell differentiation [GO:0042492], cytotoxic T cell differentiation [GO:0045065], GO:0045066, alpha-beta T cell differentiation [GO:0046632], exhausted T cell differentiation [GO:0160083] Relationships: is a type of lymphocyte differentiation [GO:0030098]; is a type of GO:0042110 Also known as: T lymphocyte differentiation, T-cell differentiation, T-lymphocyte differentiation, T cell development Sources: GOC:jid, GOC:mah, GO_REF:0000022 Note: Note that the term 'thymocyte differentiation' was merged into this term because thymocytes are T cells, and thus the term was essentially redundant. Note that immunologists typically use the word 'development' to refer to cells of B or T cell lineages undergoing the process that GO describes as 'cell differentiation'. Regulation: regulated by regulation of T cell differentiation [GO:0045580]; RO_0002212 by GO:0045581; positively regulated by positive regulation of T cell differentiation [GO:0045582] Definition: The process in which a precursor cell type acquires characteristics of a more mature T-cell. A T cell is a type of lymphocyte whose definin characteristic is the expression of a T cell receptor complex.